{
  "term_label": "sperm capacitation",
  "term_id": "GO:0048240",
  "gene": "UniProtKB:P04279",
  "gene_name": "Semenogelin-1",
  "gene_symbol": "SEMG1"
}